flavonol-3-O-triglucoside O-coumaroyltransferase activity [GO:0033811] (MF) Sources: EC:2.3.1.173 Relationships: is a type of acyltransferase activity, transferring groups other than amino-acyl groups [GO:0016747] Also known as: 4-coumaroyl-CoA:flavonol-3-O-[beta-D-glucosyl-(1->2)-beta-D-glucosyl-(1->2)-beta-D-glucoside] 6'''-O-4-coumaroyltransferase activity Definition: Catalysis of the reaction: 4-coumaroyl-CoA + a flavonol 3-O-[beta-D-glucosyl-(1->2)-beta-D-glucosyl-(1->2)-beta-D-glucoside] = CoA + a flavonol 3-O-[6-(4-coumaroyl)-beta-D-glucosyl-(1->2)-beta-D-glucosyl-(1->2)-beta-D-glucoside].